native siderophore export across plasma membrane [GO:0180061] (biological process) Relationships: is_a siderophore-dependent iron import pathway [GO:0180060] Sources: GOC:vw Definition: The directed movement of siderophores, low molecular weight Fe(III)-chelating substances, from inside of a cell, across the plasma membrane and into the extracellular region.